{
  "term_id": "UNKNOWN:0001",
  "gene": "UniProtKB:O15245",
  "term_label": "Unknown molecular function",
  "gene_name": "Solute carrier family 22 member 1",
  "gene_symbol": "SLC22A1"
}